{
  "term_id": "GO:0005886",
  "gene_symbol": "ABCC1",
  "gene": "UniProtKB:P33527",
  "term_label": "plasma membrane",
  "gene_name": "Multidrug resistance-associated protein 1"
}